{
  "term_id": "GO:0003713",
  "term_label": "transcription coactivator activity",
  "gene_name": "DDB1- and CUL4-associated factor 6",
  "gene": "UniProtKB:Q58WW2",
  "gene_symbol": "DCAF6"
}